L-tyrosine biosynthetic process, by oxidation of phenylalanine [GO:0019293] (biological process) Definition: The conversion of phenylalanine to tyrosine. References: PMID:4004813 Also known as: L-tyrosine biosynthesis IV, tyrosine anabolism, by oxidation of phenylalanine, tyrosine formation, by oxidation of phenylalanine, tyrosine synthesis, by oxidation of phenylalanine Relationships: is_a L-tyrosine biosynthetic process [GO:0006571]